{
  "gene": "UniProtKB:Q9UL25",
  "gene_symbol": "RAB21",
  "gene_name": "Ras-related protein Rab-21",
  "term_id": "GO:0005769",
  "term_label": "early endosome"
}